haustorium [GO:0085035] (cellular component) Note: See also: extrahaustorial matrix ; GO:0085036 and extrahaustorial membrane ; GO:0085037. Sources: GOC:pamgo_curators Relationships: is a type of GO:0042995 Subtypes: arbuscule [GO:0085041] Definition: A projection from a cell or tissue that penetrates the host's cell wall and invaginates the host cell membrane.